Myb complex [GO:0031523] (cellular component) Also known as: Myeloblastosis proto-oncogene protein complex References: PMID:12490953, PMID:15545624 Definition: A multisubunit complex consisting of Myb and other proteins that regulates site specific DNA replication, gene amplification and transcriptional repression. Relationships: is a type of nuclear protein-containing complex [GO:0140513]